{
  "gene_name": "Cholinephosphotransferase 1",
  "gene": "UniProtKB:Q8WUD6",
  "gene_symbol": "CHPT1",
  "term_id": "GO:0004142",
  "term_label": "diacylglycerol cholinephosphotransferase activity"
}